{
  "term_id": "GO:0000408",
  "gene_name": "EKC_KEOPS complex subunit LAGE3",
  "gene_symbol": "LAGE3",
  "term_label": "EKC/KEOPS complex",
  "gene": "UniProtKB:Q14657"
}